{
  "gene_symbol": "H3Y1",
  "gene_name": "Histone H3.Y",
  "term_id": "GO:0030527",
  "gene": "UniProtKB:P0DPK2",
  "term_label": "structural constituent of chromatin"
}